regulation of pyloric antrum smooth muscle contraction [GO:0120071] (biological process) Definition: Any process that modulates the frequency, rate or extent of any pyloric antrum smooth muscle contraction. References: PMID:15890336 Sources: GOC:sl Relationships: is a type of regulation of gastro-intestinal system smooth muscle contraction [GO:1904304]; regulates pyloric antrum smooth muscle contraction [GO:0120065] Subtypes: positive regulation of pyloric antrum smooth muscle contraction [GO:0120072], negative regulation of pyloric antrum smooth muscle contraction [GO:0120073]